{
  "gene_symbol": "CES2",
  "term_label": "Unknown cellular component",
  "gene": "UniProtKB:O00748",
  "term_id": "UNKNOWN:0003",
  "gene_name": "Cocaine esterase"
}